{
  "term_label": "endoplasmic reticulum to Golgi vesicle-mediated transport",
  "gene_symbol": "A0A2R8YE69",
  "gene": "UniProtKB:A0A2R8YE69",
  "gene_name": "Uncharacterized protein",
  "term_id": "GO:0006888"
}